{
  "gene": "UniProtKB:Q9H1P3",
  "term_label": "Unknown biological process",
  "gene_name": "Oxysterol-binding protein-related protein 2",
  "gene_symbol": "OSBPL2",
  "term_id": "UNKNOWN:0002"
}